{
  "gene_symbol": "ETS1",
  "term_id": "GO:0006357",
  "gene": "UniProtKB:P14921",
  "term_label": "regulation of transcription by RNA polymerase II",
  "gene_name": "Protein C-ets-1"
}